{
  "term_label": "DNA cytosine deamination",
  "gene_symbol": "APOBEC3F",
  "gene": "UniProtKB:Q8IUX4",
  "term_id": "GO:0070383",
  "gene_name": "DNA dC-dU-editing enzyme APOBEC-3F"
}